chondrocyte development [GO:0002063] (biological process) Subtypes: chondrocyte development involved in endochondral bone morphogenesis [GO:0003433] Regulation: regulated by regulation of chondrocyte development [GO:0061181]; negatively regulated by GO:0061182; positively regulated by GO:1902761 Relationships: is a type of cell development [GO:0048468]; is part of chondrocyte differentiation [GO:0002062] Definition: The process whose specific outcome is the progression of a chondrocyte over time, from its commitment to its mature state. Chondrocyte development does not include the steps involved in committing a chondroblast to a chondrocyte fate. Sources: GOC:dph